{
  "term_id": "GO:0035418",
  "gene_symbol": "PCLO",
  "gene_name": "Protein piccolo",
  "gene": "UniProtKB:Q9Y6V0",
  "term_label": "protein localization to synapse"
}